{
  "gene_name": "Homeobox protein Nkx-6.1",
  "gene_symbol": "NKX6-1",
  "term_label": "nucleus",
  "term_id": "GO:0005634",
  "gene": "UniProtKB:P78426"
}